{
  "term_id": "GO:0007417",
  "gene_symbol": "BCAN",
  "gene": "UniProtKB:Q96GW7",
  "term_label": "central nervous system development",
  "gene_name": "Brevican core protein"
}